{
  "term_id": "GO:0005829",
  "term_label": "cytosol",
  "gene_symbol": "EFL1",
  "gene_name": "Elongation factor-like GTPase 1",
  "gene": "UniProtKB:Q7Z2Z2"
}